{
  "gene_name": "Mitotic checkpoint protein BUB3",
  "term_id": "GO:0007094",
  "gene": "UniProtKB:O43684",
  "gene_symbol": "BUB3",
  "term_label": "mitotic spindle assembly checkpoint signaling"
}